{
  "gene": "UniProtKB:P51508",
  "gene_name": "Zinc finger protein 81",
  "term_id": "GO:0006357",
  "gene_symbol": "ZNF81",
  "term_label": "regulation of transcription by RNA polymerase II"
}